{
  "gene_name": "Lysophosphatidic acid phosphatase type 6",
  "gene": "UniProtKB:Q9NPH0",
  "term_label": "lysophosphatidic acid phosphatase activity",
  "term_id": "GO:0052642",
  "gene_symbol": "ACP6"
}